{
  "gene_symbol": "TLNRD1",
  "gene_name": "Talin rod domain-containing protein 1",
  "term_label": "actin binding",
  "term_id": "GO:0003779",
  "gene": "UniProtKB:Q9H1K6"
}